cell cortex of cell tip [GO:0051285] (cellular component) Also known as: cell cortex of cell end Definition: The region directly beneath the plasma membrane at the cell tip. The cell tip is the region at either end of the longest axis of a cylindrical or elongated cell. Sources: GOC:ai Subtypes: cell cortex of non-growing cell tip [GO:0140472], cell cortex of growing cell tip [GO:1902716] Relationships: is a type of cell cortex region [GO:0099738]; BFO_0000050 GO:0051286